{
  "term_label": "microtubule",
  "gene": "UniProtKB:Q9UJT1",
  "gene_symbol": "TUBD1",
  "gene_name": "Tubulin delta chain",
  "term_id": "GO:0005874"
}